regulation of lactation [GO:1903487] (biological process) Relationships: is a type of regulation of body fluid levels [GO:0050878]; is a type of regulation of secretion [GO:0051046]; is a type of regulation of multicellular organismal development [GO:2000026]; regulates lactation [GO:0007595] Definition: Any process that modulates the frequency, rate or extent of lactation. Subtypes: negative regulation of lactation [GO:1903488], positive regulation of lactation [GO:1903489] References: PMID:19563620 Sources: GOC:TermGenie, GOC:mr, GO_REF:0000058